plasma kallikrein-kinin cascade [GO:0002353] (biological process) Relationships: is a type of kinin cascade [GO:0002254] Definition: A series of reactions that takes place outside the cell occurring in response to tissue damage and initiated within blood plasma by the action of activated Factor XII (Hageman Factor) on prekallikrein to convert it to plasma kallikrein, and the subsequent reaction of plasma kallikrein with high molecular weight kininogen. The ultimate product of the plasma kallikrein-kinin cascade is bradykinin, an agent known to induce smooth muscle contraction, vasoconstriction, and increased vascular permeability. References: PMID:11842287, PMID:14501145 Sources: GOC:add, ISBN:0721601871 Regulation: regulated by regulation of plasma kallikrein-kinin cascade [GO:0002529]; negatively regulated by negative regulation of plasma kallikrein-kinin cascade [GO:0002549]; positively regulated by positive regulation of plasma kallikrein-kinin cascade [GO:0002550]